{
  "term_id": "GO:0051082",
  "gene_name": "Heat shock protein beta-6",
  "term_label": "unfolded protein binding",
  "gene_symbol": "HSPB6",
  "gene": "UniProtKB:O14558"
}